{
  "gene_name": "Disintegrin and metalloproteinase domain-containing protein 21",
  "gene_symbol": "ADAM21",
  "term_label": "metalloendopeptidase activity",
  "term_id": "GO:0004222",
  "gene": "UniProtKB:Q9UKJ8"
}